negative regulation of formation of symbiont germ tube hook structure for appressorium development [GO:0075032] (biological process) Relationships: is a type of negative regulation of developmental process [GO:0051093]; is a type of modulation of formation of symbiont germ tube hook structure for appressorium development [GO:0075030]; negatively regulates formation of appressorium germ tube hook structure [GO:0075029] Also known as: negative regulation of formation of symbiont germ tube hook structure on or near host, negative regulation of germ tube tip of symbiont on or near the exterior of host, negative regulation of symbiont germ tube hook structure formation on or near host Definition: Any process that stops, prevents, or reduces the frequency, rate or extent of symbiont germ tube hook structure formation. Sources: GOC:pamgo_curators